{
  "term_label": "regulation of transcription by RNA polymerase II",
  "gene_name": "Paired mesoderm homeobox protein 2A",
  "term_id": "GO:0006357",
  "gene": "UniProtKB:O14813",
  "gene_symbol": "PHOX2A"
}